{
  "term_label": "SNARE complex assembly",
  "gene": "UniProtKB:Q9P2Y5",
  "term_id": "GO:0035493",
  "gene_name": "UV radiation resistance-associated gene protein",
  "gene_symbol": "UVRAG"
}